{
  "gene_symbol": "PRICKLE1",
  "term_label": "Unknown molecular function",
  "gene": "UniProtKB:Q96MT3",
  "gene_name": "Prickle-like protein 1",
  "term_id": "UNKNOWN:0001"
}